positive regulation of transcription from RNA polymerase II promoter by a nonfermentable carbon source [GO:0061414] (biological process) Relationships: is a type of carbon catabolite activation of transcription from RNA polymerase II promoter [GO:0000436]; is a type of GO:0061413 References: PMID:19686338 Sources: GOC:dph Definition: A transcription regulation process in which the presence of a nonfermentable carbon source leads to an increase of the frequency, rate, or extent of transcription, from an RNA polymerase II promoter, of specific genes involved in the metabolism of other carbon sources.